{
  "term_label": "DNA-binding transcription factor activity, RNA polymerase II-specific",
  "gene_name": "MHC class II regulatory factor RFX1",
  "gene": "UniProtKB:P22670",
  "gene_symbol": "RFX1",
  "term_id": "GO:0000981"
}